{
  "gene": "UniProtKB:Q9P2D1",
  "gene_name": "Chromodomain-helicase-DNA-binding protein 7",
  "term_id": "GO:0007417",
  "term_label": "central nervous system development",
  "gene_symbol": "CHD7"
}